{
  "gene_symbol": "BCKDK",
  "gene": "UniProtKB:O14874",
  "term_label": "regulation of pyruvate decarboxylation to acetyl-CoA",
  "gene_name": "[3-methyl-2-oxobutanoate dehydrogenase [lipoamide]] kinase, mitochondrial",
  "term_id": "GO:0010510"
}